{
  "term_label": "C-C chemokine receptor activity",
  "gene_symbol": "CX3CR1",
  "gene_name": "CX3C chemokine receptor 1",
  "term_id": "GO:0016493",
  "gene": "UniProtKB:P49238"
}